{
  "gene": "UniProtKB:A5D8V7",
  "term_id": "GO:0036064",
  "term_label": "ciliary basal body",
  "gene_name": "Outer dynein arm-docking complex subunit 3",
  "gene_symbol": "ODAD3"
}